ErbB-4 class receptor binding [GO:1990631] (molecular function) Also known as: HER4 receptor binding Relationships: is a type of signaling receptor binding [GO:0005102] Definition: Binding to the protein-tyrosine kinase receptor ErbB-4/HER4. References: PMID:18523588 Sources: GOC:sl